{
  "gene_name": "Cyclin-dependent kinase 4 inhibitor B",
  "gene": "UniProtKB:P42772",
  "gene_symbol": "CDKN2B",
  "term_label": "negative regulation of cell population proliferation",
  "term_id": "GO:0008285"
}